{
  "gene_symbol": "PSMG4",
  "gene_name": "Proteasome assembly chaperone 4",
  "term_id": "UNKNOWN:0002",
  "term_label": "Unknown biological process",
  "gene": "UniProtKB:Q5JS54"
}